{
  "term_id": "GO:0006612",
  "gene_symbol": "ZDHHC14",
  "gene": "UniProtKB:Q8IZN3",
  "gene_name": "Palmitoyltransferase ZDHHC14",
  "term_label": "protein targeting to membrane"
}